{
  "gene_symbol": "TMTC3",
  "gene_name": "Protein O-mannosyl-transferase TMTC3",
  "gene": "UniProtKB:Q6ZXV5",
  "term_label": "mannosyltransferase activity",
  "term_id": "GO:0000030"
}